{
  "gene_symbol": "Q499Y3",
  "term_id": "UNKNOWN:0002",
  "term_label": "Unknown biological process",
  "gene": "UniProtKB:Q499Y3",
  "gene_name": "Putative uncharacterized protein C10orf88-like"
}